neuroblast development [GO:0014019] (BP) Sources: GOC:ef, ISBN:0878932585 Relationships: is a type of GO:0048468; is part of neuroblast differentiation [GO:0014016] Definition: The process aimed at the progression of a neuroblast over time, from initial commitment of the cell to a specific state, to the mature neuroblast. It does not include processes where the neuroblast turns into a glial cell or a neuron.